phytol salvage [GO:0033307] (biological process) Sources: GOC:mah, MetaCyc:PWY-5107 Also known as: phytol salvage pathway Relationships: is a type of phytol biosynthetic process [GO:0033520]; is_a metabolic compound salvage [GO:0043094] Definition: A process that generates phytol, (2E,7R,11R)-3,7,11,15-tetramethylhexadec-2-en-1-ol, from derivatives of it without de novo synthesis.